{
  "term_label": "Unknown molecular function",
  "gene": "UniProtKB:A0A0B4J241",
  "gene_name": "T cell receptor alpha variable 13-1",
  "gene_symbol": "TRAV13-1",
  "term_id": "UNKNOWN:0001"
}